ATPase-coupled ectoine transmembrane transporter activity [GO:0033286] (molecular function) Sources: GOC:mlg, RHEA:32787 Also known as: ectoine transmembrane transporter activity, ATP-dependent ectoine transmembrane transporter activity, ectoine-transporting ATPase activity Relationships: is a type of ATPase-coupled monocarboxylic acid transmembrane transporter activity [GO:0033285]; is part of ectoine transmembrane transport [GO:0051470] Definition: Enables the transfer of a solute or solutes from one side of a membrane to the other according to the reaction: ATP + H2O + ectoine(out/in) = ADP + phosphate + ectoine(in/out).